{
  "gene_name": "Caveolin-2",
  "term_id": "GO:0051480",
  "gene": "UniProtKB:P51636",
  "gene_symbol": "CAV2",
  "term_label": "regulation of cytosolic calcium ion concentration"
}